regulation of abscisic acid-activated signaling pathway [GO:0009787] (biological process) Also known as: regulation of abscisic acid mediated signalling, regulation of abscisic acid mediated signaling pathway Definition: Any process that modulates the frequency, rate or extent of abscisic acid (ABA) signaling. Relationships: is a type of regulation of signal transduction [GO:0009966]; is a type of GO:1905957; regulates abscisic acid-activated signaling pathway [GO:0009738] Sources: GOC:lr Subtypes: negative regulation of abscisic acid-activated signaling pathway [GO:0009788], positive regulation of abscisic acid-activated signaling pathway [GO:0009789]